{
  "term_label": "Unknown biological process",
  "term_id": "UNKNOWN:0002",
  "gene_symbol": "IGFL3",
  "gene_name": "Insulin growth factor-like family member 3",
  "gene": "UniProtKB:Q6UXB1"
}